{
  "term_id": "GO:0005886",
  "gene_symbol": "SLC28A3",
  "gene_name": "Solute carrier family 28 member 3",
  "term_label": "plasma membrane",
  "gene": "UniProtKB:Q9HAS3"
}